{
  "gene_symbol": "ANAPC1",
  "gene_name": "Anaphase-promoting complex subunit 1",
  "gene": "UniProtKB:Q9H1A4",
  "term_id": "GO:0007091",
  "term_label": "metaphase/anaphase transition of mitotic cell cycle"
}